establishment of localization [GO:0051234] (biological process) Sources: GOC:ai, GOC:dos Subtypes: transport [GO:0006810], establishment of protein localization [GO:0045184], establishment of RNA localization [GO:0051236], establishment of localization in cell [GO:0051649], establishment of organelle localization [GO:0051656], establishment of protein-containing complex localization to telomere [GO:0097695] Definition: Any process that localizes a substance or cellular component. This may occur via movement, tethering or selective degradation. Also known as: establishment of localisation Relationships: is a type of localization [GO:0051179]